{
  "term_id": "UNKNOWN:0001",
  "gene_name": "Voltage-dependent L-type calcium channel subunit alpha-1D",
  "term_label": "Unknown molecular function",
  "gene_symbol": "CACNA1D",
  "gene": "UniProtKB:Q01668"
}